synaptic cleft [GO:0043083] (cellular component) Definition: The narrow gap that separates the presynaptic and postsynaptic membranes, into which neurotransmitter is released. Relationships: is a type of GO:0005576 References: PMID:30784960 Sources: GOC:jl